{
  "term_label": "nucleolus",
  "gene": "UniProtKB:Q969H6",
  "term_id": "GO:0005730",
  "gene_name": "Ribonuclease P_MRP protein subunit POP5",
  "gene_symbol": "POP5"
}